{
  "term_id": "GO:0005102",
  "gene_symbol": "BTN2A1",
  "term_label": "signaling receptor binding",
  "gene_name": "Butyrophilin subfamily 2 member A1",
  "gene": "UniProtKB:Q7KYR7"
}